{
  "term_label": "nucleus",
  "gene_name": "Coiled-coil domain-containing protein 137",
  "term_id": "GO:0005634",
  "gene": "UniProtKB:Q6PK04",
  "gene_symbol": "CCDC137"
}